blood-group-substance endo-1,4-beta-galactosidase activity [GO:0033929] (molecular function) Relationships: is_a GO:0015925 Sources: EC:3.2.1.102 Also known as: endo-beta-galactosidase activity, blood-group-substance 1,4-beta-D-galactanohydrolase activity Definition: Catalysis of the endohydrolysis of (1->4)-beta-D-galactosidic linkages in blood group A and B substances.